{
  "term_id": "GO:0050778",
  "gene": "UniProtKB:P28067",
  "gene_symbol": "HLA-DMA",
  "gene_name": "HLA class II histocompatibility antigen, DM alpha chain",
  "term_label": "positive regulation of immune response"
}